{
  "gene_name": "PDZ domain-containing protein GIPC1",
  "gene": "UniProtKB:O14908",
  "term_label": "Unknown molecular function",
  "gene_symbol": "GIPC1",
  "term_id": "UNKNOWN:0001"
}